{
  "gene_symbol": "HORMAD1",
  "gene_name": "HORMA domain-containing protein 1",
  "term_id": "GO:0007130",
  "gene": "UniProtKB:Q86X24",
  "term_label": "synaptonemal complex assembly"
}